3-(3-hydroxyphenyl)propanoate biosynthetic process [GO:1901795] (biological process) Relationships: is a type of monocarboxylic acid biosynthetic process [GO:0072330] Definition: The chemical reactions and pathways resulting in the formation of 3-(3-hydroxyphenyl)propanoate. References: PMID:10537203 Sources: GOC:TermGenie, GOC:yaf Also known as: 3-(3-hydroxyphenyl)propanoate anabolism, 3-(3-hydroxyphenyl)propanoate biosynthesis, 3-(3-hydroxyphenyl)propanoate formation, 3-(3-hydroxyphenyl)propanoate synthesis